{
  "gene_name": "Integrin beta-5",
  "term_label": "cell-cell adhesion",
  "gene_symbol": "ITGB5",
  "gene": "UniProtKB:P18084",
  "term_id": "GO:0098609"
}